{
  "term_label": "Unknown molecular function",
  "term_id": "UNKNOWN:0001",
  "gene_symbol": "GAS8",
  "gene": "UniProtKB:O95995",
  "gene_name": "Dynein regulatory complex subunit 4"
}